plant endodermal cell fate specification [GO:0160057] (biological process) References: PMID:26415082 Definition: The process in which a cell becomes capable of differentiating autonomously into a plant endodermal cell in an environment that is neutral with respect to the developmental pathway. Upon specification, the cell fate can be reversed. Relationships: is a type of GO:0001708